{
  "gene_name": "Biorientation of chromosomes in cell division protein 1-like 1",
  "term_label": "replication fork processing",
  "gene_symbol": "BOD1L1",
  "term_id": "GO:0031297",
  "gene": "UniProtKB:Q8NFC6"
}